{
  "term_label": "mitochondrion",
  "gene_symbol": "TOMM34",
  "gene": "UniProtKB:Q15785",
  "term_id": "GO:0005739",
  "gene_name": "Mitochondrial import receptor subunit TOM34"
}